{
  "gene": "UniProtKB:Q4VNC0",
  "term_label": "polyamine transmembrane transporter activity",
  "gene_symbol": "ATP13A5",
  "gene_name": "Probable cation-transporting ATPase 13A5",
  "term_id": "GO:0015203"
}